cellular response to methamphetamine hydrochloride [GO:1904314] (biological process) Also known as: cellular response to methamphetamine HCL Definition: Any process that results in a change in state or activity of a cell (in terms of movement, secretion, enzyme production, gene expression, etc.) as a result of a methamphetamine hydrochloride stimulus. Relationships: is a type of cellular response to amine stimulus [GO:0071418]; is a type of response to methamphetamine hydrochloride [GO:1904313] References: PMID:22174933 Sources: GOC:TermGenie, GO_REF:0000071